{
  "gene": "UniProtKB:Q7L3B6",
  "gene_name": "Hsp90 co-chaperone Cdc37-like 1",
  "term_label": "protein-folding chaperone binding",
  "term_id": "GO:0051087",
  "gene_symbol": "CDC37L1"
}